{
  "term_label": "transmembrane transport",
  "gene_symbol": "ABCC8",
  "gene_name": "ATP-binding cassette sub-family C member 8",
  "term_id": "GO:0055085",
  "gene": "UniProtKB:Q09428"
}